{
  "term_id": "GO:0005886",
  "gene": "UniProtKB:A0A599",
  "gene_symbol": "TRBV5-6",
  "gene_name": "T cell receptor beta variable 5-6",
  "term_label": "plasma membrane"
}